{
  "gene_name": "Protein Wnt-16",
  "gene_symbol": "WNT16",
  "term_id": "GO:0030182",
  "gene": "UniProtKB:Q9UBV4",
  "term_label": "neuron differentiation"
}